{
  "gene_symbol": "DNASE1",
  "term_id": "GO:0006308",
  "gene_name": "Deoxyribonuclease-1",
  "term_label": "DNA catabolic process",
  "gene": "UniProtKB:P24855"
}